negative regulation of phosphorus metabolic process [GO:0010563] (biological process) Relationships: is a type of negative regulation of metabolic process [GO:0009892]; is a type of regulation of phosphorus metabolic process [GO:0051174]; negatively regulates phosphorus metabolic process [GO:0006793] Subtypes: negative regulation of phosphate metabolic process [GO:0045936], negative regulation of phosphorus utilization [GO:0045942], GO:1900975 Sources: GOC:dph, GOC:tb Definition: Any process that decreases the frequency, rate or extent of the chemical reactions and pathways involving phosphorus or compounds containing phosphorus.